ligand-modulated transcription repressor activity [GO:0141096] (molecular function) Also known as: ligand-activated transcription repressor activity Definition: A DNA-binding transcription repressor activity regulated by binding to a ligand and that inhibits the transcription of specific genes and gene sets. References: PMID:21555518 Relationships: is a type of DNA-binding transcription repressor activity [GO:0001217]; is a type of ligand-modulated transcription factor activity [GO:0098531]